CMP-N-acetylneuraminate transmembrane transport [GO:0015782] (biological process) Definition: The directed movement of CMP-N-acetylneuraminate into, out of or within a cell, or between cells, by means of some agent such as a transporter or pore. Sources: GOC:ai Also known as: CMP-sialic acid transport, CMP-N-acetylneuraminate transport Relationships: is a type of organic anion transport [GO:0015711]; is a type of GO:0090481